{
  "gene_symbol": "PDE4D",
  "term_id": "UNKNOWN:0003",
  "term_label": "Unknown cellular component",
  "gene": "UniProtKB:Q08499",
  "gene_name": "cAMP-specific 3',5'-cyclic phosphodiesterase 4D"
}